positive regulation of mast cell proliferation [GO:0070668] (biological process) Relationships: is a type of positive regulation of leukocyte proliferation [GO:0070665]; is a type of regulation of mast cell proliferation [GO:0070666]; positively regulates mast cell proliferation [GO:0070662] Sources: GOC:add, GOC:mah Definition: Any process that activates or increases the rate or extent of mast cell proliferation. Also known as: up regulation of mast cell proliferation, up-regulation of mast cell proliferation, upregulation of mast cell proliferation, activation of mast cell proliferation, stimulation of mast cell proliferation